{
  "term_id": "UNKNOWN:0002",
  "gene_symbol": "ITIH3",
  "gene": "UniProtKB:Q06033",
  "gene_name": "Inter-alpha-trypsin inhibitor heavy chain H3",
  "term_label": "Unknown biological process"
}